response to trehalose-6-phosphate [GO:0080094] (biological process) Subtypes: cellular response to trehalose-6-phosphate stimulus [GO:0071330] Relationships: is a type of response to organophosphorus [GO:0046683]; is a type of response to oxygen-containing compound [GO:1901700] Definition: Any process that results in a change in state or activity of a cell or an organism (in terms of movement, secretion, enzyme production, gene expression, etc.) as a result of a trehalose-6-phosphate stimulus. References: PMID:19193861 Also known as: response to trehalose-6-phosphate stimulus